{
  "term_id": "GO:0000045",
  "gene_name": "Tumor protein p53-inducible nuclear protein 1",
  "term_label": "autophagosome assembly",
  "gene_symbol": "TP53INP1",
  "gene": "UniProtKB:Q96A56"
}